{
  "term_id": "GO:0030272",
  "term_label": "5-formyltetrahydrofolate cyclo-ligase activity",
  "gene_symbol": "MTHFS",
  "gene_name": "5-formyltetrahydrofolate cyclo-ligase",
  "gene": "UniProtKB:P49914"
}